negative regulation of establishment of T cell polarity [GO:1903904] (BP) Definition: Any process that stops, prevents or reduces the frequency, rate or extent of establishment of T cell polarity. Relationships: is a type of negative regulation of T cell activation [GO:0050868]; is a type of GO:1903903; negatively regulates establishment of T cell polarity [GO:0001768] Also known as: down regulation of T cell polarization, down regulation of T lymphocyte polarization, down regulation of T-cell polarization, down regulation of establishment of T cell polarity, down regulation of establishment of T lymphocyte polarity, down regulation of establishment of T-cell polarity, down regulation of establishment of T-lymphocyte polarity, down-regulation of T cell polarization, down-regulation of T lymphocyte polarization, down-regulation of T-cell polarization, down-regulation of establishment of T cell polarity, down-regulation of establishment of T lymphocyte polarity, down-regulation of establishment of T-cell polarity, down-regulation of establishment of T-lymphocyte polarity, downregulation of T cell polarization, downregulation of T lymphocyte polarization, downregulation of T-cell polarization, downregulation of establishment of T cell polarity, downregulation of establishment of T lymphocyte polarity, downregulation of establishment of T-cell polarity, downregulation of establishment of T-lymphocyte polarity, negative regulation of T cell polarization, negative regulation of T lymphocyte polarization, negative regulation of T-cell polarization, negative regulation of establishment of T lymphocyte polarity, negative regulation of establishment of T-cell polarity, negative regulation of establishment of T-lymphocyte polarity, inhibition of T cell polarization, inhibition of T lymphocyte polarization, inhibition of T-cell polarization, inhibition of establishment of T cell polarity, inhibition of establishment of T lymphocyte polarity, inhibition of establishment of T-cell polarity, inhibition of establishment of T-lymphocyte polarity References: PMID:23575248 Sources: GOC:TermGenie, GOC:als, GO_REF:0000058